{
  "gene": "UniProtKB:Q15111",
  "gene_symbol": "PLCL1",
  "term_id": "GO:0051209",
  "term_label": "release of sequestered calcium ion into cytosol",
  "gene_name": "Inactive phospholipase C-like protein 1"
}